regulation of PERK-mediated unfolded protein response [GO:1903897] (BP) References: PMID:22013210 Sources: GOC:PARL, GOC:TermGenie, GOC:bf, GO_REF:0000058 Relationships: is a type of regulation of endoplasmic reticulum unfolded protein response [GO:1900101]; regulates PERK-mediated unfolded protein response [GO:0036499] Subtypes: negative regulation of PERK-mediated unfolded protein response [GO:1903898], positive regulation of PERK-mediated unfolded protein response [GO:1903899] Definition: Any process that modulates the frequency, rate or extent of the PERK-mediated unfolded protein response. Also known as: regulation of PERK signal transduction pathway, regulation of PERK branch of UPR, regulation of PKR-like ER kinase signal transduction, regulation of UPR signaling by PERK stress sensor, regulation of endoplasmic reticulum unfolded protein response; PERK signaling, regulation of EIF2AK3-mediated unfolded protein response, regulation of PERK signaling in response to endoplasmic reticulum stress